tRNA (5-carboxymethylaminomethyluridine(34)-2'-O)-methyltransferase activity [GO:0141102] (molecular function) Definition: Catalysis of the reaction: 5-carboxymethylaminomethyluridine34 in tRNA(Leu) + S-adenosyl-L-methionine = 5-carboxymethylaminomethyl-2'-O-methyluridine34 in tRNA(Leu) + H+ + S-adenosyl-L-homocysteine. References: PMID:20855540 Sources: RHEA:43088 Also known as: tRNA (cytidine(34)/5-carboxymethylaminomethyluridine(34)-2'-O)- methyltransferase activity Relationships: is a type of GO:0016300